{
  "term_id": "GO:0005096",
  "term_label": "GTPase activator activity",
  "gene_symbol": "RACGAP1",
  "gene": "UniProtKB:Q9H0H5",
  "gene_name": "Rac GTPase-activating protein 1"
}